{
  "gene_symbol": "MYO6",
  "gene": "UniProtKB:Q9UM54",
  "term_label": "cytoplasm",
  "gene_name": "Unconventional myosin-VI",
  "term_id": "GO:0005737"
}